{
  "gene": "UniProtKB:Q9P2B4",
  "term_id": "GO:1903119",
  "gene_symbol": "CTTNBP2NL",
  "gene_name": "CTTNBP2 N-terminal-like protein",
  "term_label": "protein localization to actin cytoskeleton"
}